{
  "term_label": "extracellular space",
  "term_id": "GO:0005615",
  "gene": "UniProtKB:Q5W188",
  "gene_symbol": "CST9LP1",
  "gene_name": "Putative cystatin-9-like protein CST9LP1"
}